{
  "term_label": "sodium-independent organic anion transport",
  "gene_symbol": "SLCO1B1",
  "gene_name": "Solute carrier organic anion transporter family member 1B1",
  "gene": "UniProtKB:Q9Y6L6",
  "term_id": "GO:0043252"
}